{
  "term_label": "regulation of transcription by RNA polymerase II",
  "gene_name": "Homeobox protein Nkx-3.2",
  "gene": "UniProtKB:P78367",
  "gene_symbol": "NKX3-2",
  "term_id": "GO:0006357"
}